{
  "gene": "UniProtKB:Q96AQ8",
  "gene_symbol": "MCUR1",
  "term_label": "calcium import into the mitochondrion",
  "gene_name": "Mitochondrial calcium uniporter regulator 1",
  "term_id": "GO:0036444"
}